{
  "term_id": "GO:1901612",
  "gene_name": "Pleckstrin homology domain-containing family N member 1",
  "term_label": "cardiolipin binding",
  "gene": "UniProtKB:Q494U1",
  "gene_symbol": "PLEKHN1"
}